{
  "gene_name": "Glycerate kinase",
  "term_label": "cytoplasm",
  "gene": "UniProtKB:Q8IVS8",
  "term_id": "GO:0005737",
  "gene_symbol": "GLYCTK"
}